positive regulation of cell motility [GO:2000147] (BP) Definition: Any process that activates or increases the frequency, rate or extent of cell motility. Sources: GOC:mah Relationships: is a type of positive regulation of locomotion [GO:0040017]; is a type of positive regulation of cellular process [GO:0048522]; is a type of regulation of cell motility [GO:2000145]; positively regulates GO:0048870 Subtypes: positive regulation of cell migration [GO:0030335], positive regulation of amoeboid sperm motility [GO:1905418], GO:2000155 Also known as: positive regulation of cell locomotion, positive regulation of movement of a cell, positive regulation of cell movement